{
  "gene_name": "Endogenous retrovirus group K member 6 Pol protein",
  "term_id": "GO:0035613",
  "gene_symbol": "ERVK-6",
  "term_label": "RNA stem-loop binding",
  "gene": "UniProtKB:Q9BXR3"
}